regulation of shell calcification [GO:1905648] (biological process) References: PMID:14648763 Sources: GOC:TermGenie, GO_REF:0000058 Subtypes: GO:1905649, positive regulation of shell calcification [GO:1905650] Relationships: is a type of regulation of biomineral tissue development [GO:0070167]; regulates GO:0031215 Definition: Any process that modulates the frequency, rate or extent of shell calcification.